{
  "term_label": "cytoplasm",
  "gene": "UniProtKB:Q9Y285",
  "gene_name": "Phenylalanine--tRNA ligase alpha subunit",
  "term_id": "GO:0005737",
  "gene_symbol": "FARSA"
}